{
  "gene_symbol": "SLC26A7",
  "term_label": "plasma membrane",
  "term_id": "GO:0005886",
  "gene_name": "Anion exchange transporter",
  "gene": "UniProtKB:Q8TE54"
}